{
  "term_label": "plasma membrane",
  "gene": "UniProtKB:Q99795",
  "gene_name": "Cell surface A33 antigen",
  "term_id": "GO:0005886",
  "gene_symbol": "GPA33"
}